negative regulation of cytotoxic T cell degranulation [GO:0043318] (biological process) Sources: ISBN:0781735149 Definition: Any process that stops, prevents, or reduces the rate of cytotoxic T cell degranulation. Relationships: is a type of GO:0001915; is a type of negative regulation of leukocyte degranulation [GO:0043301]; is_a GO:0043317; negatively regulates cytotoxic T cell degranulation [GO:0043316] Also known as: down regulation of cytotoxic T cell degranulation, down-regulation of cytotoxic T cell degranulation, downregulation of cytotoxic T cell degranulation, negative regulation of cytotoxic T cell granule exocytosis, negative regulation of cytotoxic T lymphocyte degranulation, negative regulation of cytotoxic T lymphocyte granule exocytosis, negative regulation of cytotoxic T-cell degranulation, negative regulation of cytotoxic T-cell granule exocytosis, negative regulation of cytotoxic T-lymphocyte degranulation, negative regulation of cytotoxic T-lymphocyte granule exocytosis, inhibition of cytotoxic T cell degranulation